GDP biosynthetic process [GO:0046711] (BP) Also known as: GDP anabolism, GDP biosynthesis, GDP formation, GDP synthesis Sources: GOC:ai Definition: The chemical reactions and pathways resulting in the formation of GDP, guanosine 5'-diphosphate. Relationships: is a type of purine ribonucleotide biosynthetic process [GO:0009152]; is a type of purine ribonucleoside diphosphate biosynthetic process [GO:0009180]; is a type of GDP metabolic process [GO:0046710]